{
  "gene_symbol": "MAFA",
  "gene": "UniProtKB:Q8NHW3",
  "term_id": "GO:0006357",
  "gene_name": "Transcription factor MafA",
  "term_label": "regulation of transcription by RNA polymerase II"
}